{
  "gene_symbol": "REC8",
  "term_label": "chromatin binding",
  "gene": "UniProtKB:O95072",
  "term_id": "GO:0003682",
  "gene_name": "Meiotic recombination protein REC8 homolog"
}